{
  "gene": "UniProtKB:P01709",
  "term_label": "immune response",
  "term_id": "GO:0006955",
  "gene_name": "Immunoglobulin lambda variable 2-8",
  "gene_symbol": "IGLV2-8"
}